{
  "gene": "UniProtKB:Q9BQQ7",
  "gene_symbol": "RTP3",
  "term_id": "GO:0005737",
  "term_label": "cytoplasm",
  "gene_name": "Receptor-transporting protein 3"
}